{
  "gene": "UniProtKB:Q6X784",
  "term_label": "acrosomal vesicle",
  "term_id": "GO:0001669",
  "gene_name": "Zona pellucida-binding protein 2",
  "gene_symbol": "ZPBP2"
}